{
  "term_id": "GO:0006357",
  "gene_name": "Krueppel-like factor 3",
  "term_label": "regulation of transcription by RNA polymerase II",
  "gene_symbol": "KLF3",
  "gene": "UniProtKB:P57682"
}